{
  "term_id": "GO:0045505",
  "term_label": "dynein intermediate chain binding",
  "gene_symbol": "DYNLT2B",
  "gene": "UniProtKB:Q8WW35",
  "gene_name": "Dynein light chain Tctex-type protein 2B"
}